{
  "gene_symbol": "TTYH1",
  "gene": "UniProtKB:Q9H313",
  "term_id": "GO:0030868",
  "gene_name": "Protein tweety homolog 1",
  "term_label": "smooth endoplasmic reticulum membrane"
}